membrane repolarization during ventricular cardiac muscle cell action potential [GO:0098915] (biological process) Regulation: regulated by regulation of membrane repolarization during ventricular cardiac muscle cell action potential [GO:1905024]; negatively regulated by negative regulation of membrane repolarization during ventricular cardiac muscle cell action potential [GO:1905025]; RO_0002213 by GO:1905026 Sources: GOC:BHF, GOC:dph, GOC:mtg_cardiac_conduct_nov11, GOC:tb Relationships: is a type of membrane repolarization during cardiac muscle cell action potential [GO:0086013]; is a type of ventricular cardiac muscle cell membrane repolarization [GO:0099625]; is part of ventricular cardiac muscle cell action potential [GO:0086005] Definition: The process in which ions are transported across a membrane such that the ventricular cardiomyocyte membrane potential changes in the direction from the positive membrane potential at the peak of the action potential towards the negative resting potential. Also known as: electrocardiogram T wave, regulation of ventricular cardiac muscle repolarization, ventricular repolarization